{
  "gene_symbol": "PXDC1",
  "gene_name": "PX domain-containing protein 1",
  "term_label": "Unknown cellular component",
  "term_id": "UNKNOWN:0003",
  "gene": "UniProtKB:Q5TGL8"
}